{
  "gene_name": "TRPM8 channel-associated factor 1",
  "term_id": "GO:1901529",
  "term_label": "positive regulation of anion channel activity",
  "gene_symbol": "TCAF1",
  "gene": "UniProtKB:Q9Y4C2"
}